{
  "gene": "UniProtKB:P51957",
  "gene_name": "Serine_threonine-protein kinase Nek4",
  "term_label": "cytosol",
  "gene_symbol": "NEK4",
  "term_id": "GO:0005829"
}